positive regulation of plasma membrane repair [GO:1905686] (biological process) Definition: Any process that activates or increases the frequency, rate or extent of plasma membrane repair. References: PMID:22940583 Sources: GOC:TermGenie, GOC:bhm, GO_REF:0000058 Also known as: up regulation of plasma membrane repair, up-regulation of plasma membrane repair, upregulation of plasma membrane repair, activation of plasma membrane repair Relationships: is a type of positive regulation of cellular component organization [GO:0051130]; is_a regulation of plasma membrane repair [GO:1905684]; positively regulates plasma membrane repair [GO:0001778]